{
  "term_id": "GO:0006955",
  "gene_symbol": "IL18",
  "gene": "UniProtKB:Q14116",
  "gene_name": "Interleukin-18",
  "term_label": "immune response"
}